{
  "gene_symbol": "BID",
  "term_label": "positive regulation of release of cytochrome c from mitochondria",
  "gene_name": "BH3-interacting domain death agonist",
  "term_id": "GO:0090200",
  "gene": "UniProtKB:P55957"
}